{
  "gene": "UniProtKB:Q9UHG0",
  "gene_name": "Doublecortin domain-containing protein 2",
  "gene_symbol": "DCDC2",
  "term_id": "GO:0005815",
  "term_label": "microtubule organizing center"
}